{
  "gene_name": "DENN domain-containing protein 2D",
  "term_id": "GO:0005654",
  "term_label": "nucleoplasm",
  "gene": "UniProtKB:Q9H6A0",
  "gene_symbol": "DENND2D"
}